sepal formation [GO:0048453] (biological process) Relationships: is a type of floral organ formation [GO:0048449]; is part of sepal morphogenesis [GO:0048447] Definition: The process that gives rise to the sepal. This process pertains to the initial formation of a structure from unspecified parts. Sources: GOC:jid